{
  "gene_symbol": "GSC",
  "term_id": "GO:0000978",
  "gene_name": "Homeobox protein goosecoid",
  "gene": "UniProtKB:P56915",
  "term_label": "RNA polymerase II cis-regulatory region sequence-specific DNA binding"
}